{
  "term_id": "GO:0005667",
  "term_label": "transcription regulator complex",
  "gene_symbol": "TLE3",
  "gene_name": "Transducin-like enhancer protein 3",
  "gene": "UniProtKB:Q04726"
}